{
  "gene": "UniProtKB:Q96FA7",
  "gene_name": "Putative protein ZBED10P",
  "gene_symbol": "ZBED10P",
  "term_label": "Unknown cellular component",
  "term_id": "UNKNOWN:0003"
}